ficolin-1-rich granule membrane [GO:0101003] (cellular component) Relationships: is a type of GO:0030667; is part of GO:0070820; is part of ficolin-1-rich granule [GO:0101002] Definition: The lipid bilayer surrounding a ficolin-1-rich granule. References: PMID:23650620 Sources: GOC:mec